{
  "gene_name": "Translocation protein SEC62",
  "term_id": "GO:0008320",
  "gene": "UniProtKB:Q99442",
  "gene_symbol": "SEC62",
  "term_label": "protein transmembrane transporter activity"
}